{
  "gene_name": "C-type lectin domain family 10 member A",
  "gene": "UniProtKB:Q8IUN9",
  "gene_symbol": "CLEC10A",
  "term_id": "GO:0038187",
  "term_label": "pattern recognition receptor activity"
}